{
  "gene_name": "Serine_threonine-protein phosphatase 2A 55 kDa regulatory subunit B gamma isoform",
  "gene": "UniProtKB:Q9Y2T4",
  "term_id": "GO:0019888",
  "term_label": "protein phosphatase regulator activity",
  "gene_symbol": "PPP2R2C"
}